{
  "term_label": "nucleus",
  "gene": "UniProtKB:P57052",
  "gene_name": "Splicing regulator RBM11",
  "term_id": "GO:0005634",
  "gene_symbol": "RBM11"
}